{
  "gene_name": "Ras-interacting protein 1",
  "gene": "UniProtKB:Q5U651",
  "term_label": "cell-cell junction",
  "gene_symbol": "RASIP1",
  "term_id": "GO:0005911"
}